{
  "gene_name": "Parvalbumin-like EF-hand-containing protein",
  "gene": "UniProtKB:A0A1B0GWK0",
  "gene_symbol": "PVALEF",
  "term_label": "troponin complex",
  "term_id": "GO:0005861"
}